dolichyl-phosphate beta-D-mannosyltransferase activity [GO:0004582] (molecular function) Sources: EC:2.4.1.83 Also known as: DPM synthase activity, dolichol-phosphate-mannose synthase activity, GDP-mannose-dolichol phosphate mannosyltransferase activity, GDP-mannose:dolichyl-phosphate beta-D-mannosyltransferase activity, GDPMan:DolP mannosyltransferase activity, GDPmannose-dolichylmonophosphate mannosyltransferase activity, GDPmannose:dolichyl-phosphate mannosyltransferase activity, dolichol phosphate mannose synthase activity, dolichol-phosphate mannose synthase activity, dolichol-phosphate mannosyltransferase activity, dolichyl mannosyl phosphate synthase activity, dolichyl phosphate mannosyltransferase activity, dolichyl-phosphate mannose synthase activity, dolichyl-phospho-mannose synthase activity, guanosine diphosphomannose-dolichol phosphate mannosyltransferase activity, mannosylphosphodolichol synthase activity, mannosylphosphoryldolichol synthase activity Definition: Catalysis of the reaction: GDP-mannose + dolichyl phosphate = GDP + dolichyl D-mannosyl phosphate. Relationships: is a type of mannosyltransferase activity [GO:0000030]